{
  "term_label": "autophagosome",
  "gene_name": "Tumor protein p53-inducible nuclear protein 1",
  "term_id": "GO:0005776",
  "gene": "UniProtKB:Q96A56",
  "gene_symbol": "TP53INP1"
}